{
  "term_id": "UNKNOWN:0003",
  "gene_symbol": "PSG8",
  "term_label": "Unknown cellular component",
  "gene_name": "Pregnancy-specific beta-1-glycoprotein 8",
  "gene": "UniProtKB:Q9UQ74"
}